negative regulation of type B pancreatic cell development [GO:2000077] (biological process) Sources: GOC:obol, GOC:yaf Definition: Any process that stops, prevents, or reduces the frequency, rate or extent of pancreatic B cell development. Relationships: is_a negative regulation of cell development [GO:0010721]; is a type of GO:0051241; is_a regulation of type B pancreatic cell development [GO:2000074]; RO_0002212 type B pancreatic cell development [GO:0003323] Also known as: negative regulation of pancreatic B cell development, negative regulation of pancreatic beta cell development